developmental maturation [GO:0021700] (BP) Relationships: is a type of developmental process [GO:0032502] Definition: A developmental process, independent of morphogenetic (shape) change, that is required for an anatomical structure, cell or cellular component to attain its fully functional state. Subtypes: GO:0007593, pollen maturation [GO:0010152], seed maturation [GO:0010431], GO:0016188, pigment granule maturation [GO:0048757], synapse maturation [GO:0060074], anatomical structure maturation [GO:0071695] Sources: GOC:cls, GOC:dgh, GOC:dph, GOC:jid, GO_REF:0000021